{
  "term_id": "GO:0000932",
  "gene": "UniProtKB:Q8IU60",
  "term_label": "P-body",
  "gene_name": "m7GpppN-mRNA hydrolase",
  "gene_symbol": "DCP2"
}